{
  "gene_name": "CKLF-like MARVEL transmembrane domain-containing protein 5",
  "gene_symbol": "CMTM5",
  "gene": "UniProtKB:Q96DZ9",
  "term_label": "membrane",
  "term_id": "GO:0016020"
}